PH domain binding [GO:0042731] (molecular function) Definition: Binding to a PH domain (pleckstrin homology) of a protein, a domain of about 100 residues that occurs in a wide range of proteins involved in intracellular signaling or as constituents of the cytoskeleton. Relationships: is a type of protein domain specific binding [GO:0019904] Sources: GOC:jl, Pfam:PF00169